{
  "gene_symbol": "MIPOL1",
  "term_label": "Unknown cellular component",
  "term_id": "UNKNOWN:0003",
  "gene": "UniProtKB:Q8TD10",
  "gene_name": "Mirror-image polydactyly gene 1 protein"
}